positive regulation of actin filament binding [GO:1904531] (biological process) Definition: Any process that activates or increases the frequency, rate or extent of actin filament binding. References: PMID:24520051 Sources: GOC:TermGenie, GOC:als, GO_REF:0000059 Relationships: is a type of positive regulation of protein binding [GO:0032092]; positively regulates GO:0051015 Also known as: positive regulation of F-actin binding, up regulation of F-actin binding, up regulation of actin filament binding, up-regulation of F-actin binding, up-regulation of actin filament binding, upregulation of F-actin binding, upregulation of actin filament binding, activation of F-actin binding, activation of actin filament binding, activation of actin cross-linking activity, positive regulation of actin cross-linking activity, up regulation of actin cross-linking activity, up-regulation of actin cross-linking activity, upregulation of actin cross-linking activity